{
  "term_label": "protein-macromolecule adaptor activity",
  "gene_name": "SH2 domain-containing protein 4A",
  "term_id": "GO:0030674",
  "gene": "UniProtKB:Q9H788",
  "gene_symbol": "SH2D4A"
}